{
  "term_label": "chromatin remodeling",
  "term_id": "GO:0006338",
  "gene": "UniProtKB:Q9NVD3",
  "gene_symbol": "SETD4",
  "gene_name": "SET domain-containing protein 4"
}